{
  "gene": "UniProtKB:Q8N5I2",
  "gene_symbol": "ARRDC1",
  "gene_name": "Arrestin domain-containing protein 1",
  "term_label": "Unknown biological process",
  "term_id": "UNKNOWN:0002"
}